{
  "term_label": "mRNA binding",
  "gene_name": "YTH domain-containing protein 1",
  "gene_symbol": "YTHDC1",
  "gene": "UniProtKB:Q96MU7",
  "term_id": "GO:0003729"
}